regulation of establishment of bipolar cell polarity regulating cell shape [GO:0061160] (biological process) Sources: GOC:dph, GOC:vw Definition: Any process that modulates the rate, frequency or extent of the establishment of bipolar cell polarity that contributes to the shape of a cell. Subtypes: positive regulation of establishment of bipolar cell polarity regulating cell shape [GO:0061161] Relationships: is a type of regulation of establishment of bipolar cell polarity [GO:0061172]; is a type of regulation of establishment or maintenance of bipolar cell polarity regulating cell shape [GO:2000100]